{
  "term_label": "keratin filament",
  "term_id": "GO:0045095",
  "gene": "UniProtKB:Q15323",
  "gene_symbol": "KRT31",
  "gene_name": "Keratin, type I cuticular Ha1"
}